{
  "gene": "UniProtKB:Q99456",
  "term_id": "GO:0002009",
  "gene_name": "Keratin, type I cytoskeletal 12",
  "term_label": "morphogenesis of an epithelium",
  "gene_symbol": "KRT12"
}